{
  "term_id": "UNKNOWN:0003",
  "term_label": "Unknown cellular component",
  "gene_symbol": "BBS12",
  "gene_name": "Bardet-Biedl syndrome 12 protein",
  "gene": "UniProtKB:Q6ZW61"
}